{
  "gene_name": "Monocyte differentiation antigen CD14",
  "gene": "UniProtKB:P08571",
  "term_id": "GO:0046696",
  "term_label": "lipopolysaccharide receptor complex",
  "gene_symbol": "CD14"
}